{
  "gene_name": "snRNA-activating protein complex subunit 2",
  "term_id": "GO:0016604",
  "term_label": "nuclear body",
  "gene_symbol": "SNAPC2",
  "gene": "UniProtKB:Q13487"
}